{
  "gene_symbol": "SEMA4C",
  "gene": "UniProtKB:Q9C0C4",
  "term_label": "chemorepellent activity",
  "gene_name": "Semaphorin-4C",
  "term_id": "GO:0045499"
}